beta-D-galactose-importing ATPase activity [GO:0102014] (molecular function) Sources: RHEA:30011 Relationships: is a type of GO:0015407 Definition: Catalysis of the reaction: ATP(4-) + beta-D-galactoside + H2O = ADP(3-) + hydrogenphosphate + beta-D-galactoside + H+.